{
  "term_id": "GO:0005634",
  "gene_name": "Zinc finger and BTB domain-containing protein 16",
  "gene_symbol": "ZBTB16",
  "term_label": "nucleus",
  "gene": "UniProtKB:Q05516"
}